regulation of fungal-type cell wall beta-glucan biosynthetic process [GO:0090093] (biological process) Subtypes: regulation of ascospore wall beta-glucan biosynthetic process [GO:0060622] Sources: GOC:dph, GOC:tb Definition: Any process that modulates the frequency, rate or extent of fungal-type cell wall beta-glucan biosynthesis, the chemical reactions and pathways resulting in the formation of beta-glucans, compounds composed of glucose residues linked by beta-D-glucosidic bonds, found in the walls of fungal cells. Relationships: is_a regulation of cell wall macromolecule metabolic process [GO:0010981]; is a type of regulation of beta-glucan biosynthetic process [GO:0032951]; is a type of GO:0032995; regulates fungal-type cell wall beta-glucan biosynthetic process [GO:0070880]